response to chloroquine [GO:1902349] (biological process) References: PMID:23922869 Sources: GOC:TermGenie, GOC:kmv Subtypes: cellular response to chloroquine [GO:1902350] Definition: Any process that results in a change in state or activity of a cell or an organism (in terms of movement, secretion, enzyme production, gene expression, etc.) as a result of a chloroquine stimulus. Relationships: is a type of GO:1901698